{
  "term_id": "GO:0004001",
  "gene_symbol": "ADK",
  "gene": "UniProtKB:P55263",
  "gene_name": "Adenosine kinase",
  "term_label": "adenosine kinase activity"
}